protein linear polyubiquitination [GO:0097039] (biological process) Regulation: RO_0002211 by regulation of protein linear polyubiquitination [GO:1902528]; negatively regulated by negative regulation of protein linear polyubiquitination [GO:1902529]; positively regulated by positive regulation of protein linear polyubiquitination [GO:1902530] Also known as: M1 linkage Definition: A protein ubiquitination process in which a linear polymer of ubiquitin, formed by the amino-terminal methionine (M1) of one ubiquitin molecule and by the carboxy-terminal glycine (G76) of the next, is added to a protein. Relationships: is a type of protein polyubiquitination [GO:0000209] References: PMID:21455173, PMID:21455180, PMID:21455181, PMID:31998699 Sources: GOC:jsg, GOC:sp